{
  "gene_symbol": "SAMD5",
  "gene_name": "Sterile alpha motif domain-containing protein 5",
  "term_id": "GO:1902531",
  "gene": "UniProtKB:Q5TGI4",
  "term_label": "regulation of intracellular signal transduction"
}